pteridine catabolic process [GO:0019990] (BP) Definition: The chemical reactions and pathways resulting in the breakdown of pteridine, pyrazino(2,3-dipyrimidine), the parent structure of pterins and the pteroyl group. Sources: ISBN:0198506732 Also known as: pteridine breakdown, pteridine catabolism, pteridine degradation Relationships: is a type of pteridine metabolic process [GO:0019889]; is a type of pteridine-containing compound catabolic process [GO:0042560]